UMP biosynthetic process [GO:0006222] (biological process) Definition: The chemical reactions and pathways resulting in the formation of UMP, uridine monophosphate. Sources: ISBN:0198506732 Also known as: UMP anabolism, UMP biosynthesis, UMP formation, UMP synthesis Relationships: is a type of pyrimidine ribonucleoside monophosphate biosynthetic process [GO:0009174]; is a type of pyrimidine ribonucleotide biosynthetic process [GO:0009220]; is_a UMP metabolic process [GO:0046049] Subtypes: 'de novo' UMP biosynthetic process [GO:0044205], UMP salvage [GO:0044206]